{
  "gene_name": "Serine_threonine-protein kinase PRP4 homolog",
  "gene": "UniProtKB:Q13523",
  "term_label": "nucleus",
  "term_id": "GO:0005634",
  "gene_symbol": "PRPF4B"
}